{
  "gene_symbol": "TFEC",
  "gene": "UniProtKB:O14948",
  "term_label": "nucleus",
  "term_id": "GO:0005634",
  "gene_name": "Transcription factor EC"
}